{
  "term_id": "UNKNOWN:0001",
  "gene_symbol": "FAM184A",
  "gene_name": "Protein FAM184A",
  "gene": "UniProtKB:Q8NB25",
  "term_label": "Unknown molecular function"
}